3-keto-5-aminohexanoate cleavage activity [GO:0043720] (molecular function) Relationships: is a type of acyltransferase activity, transferring groups other than amino-acyl groups [GO:0016747] Definition: Catalysis of the reaction: 3-keto-5-aminohexanoate + acetyl-CoA = L-3-aminobutyryl-CoA + acetoacetate. Also known as: 3-keto-5-aminohexanoate cleavage enzyme References: PMID:13064 Sources: MetaCyc:R125-RXN